{
  "gene": "UniProtKB:Q460N3",
  "gene_symbol": "PARP15",
  "gene_name": "Protein mono-ADP-ribosyltransferase PARP15",
  "term_label": "negative regulation of gene expression",
  "term_id": "GO:0010629"
}